{
  "term_label": "Unknown molecular function",
  "gene": "UniProtKB:Q9HB09",
  "gene_name": "Bcl-2-like protein 12",
  "term_id": "UNKNOWN:0001",
  "gene_symbol": "BCL2L12"
}